{
  "term_label": "RNA polymerase II cis-regulatory region sequence-specific DNA binding",
  "gene": "UniProtKB:P12525",
  "gene_name": "Putative myc-like protein MYCLP1",
  "gene_symbol": "MYCLP1",
  "term_id": "GO:0000978"
}